{
  "gene_name": "C-type lectin domain family 14 member A",
  "gene_symbol": "CLEC14A",
  "term_id": "GO:0009897",
  "gene": "UniProtKB:Q86T13",
  "term_label": "external side of plasma membrane"
}